{
  "gene": "UniProtKB:P31415",
  "gene_symbol": "CASQ1",
  "term_id": "GO:0005509",
  "gene_name": "Calsequestrin-1",
  "term_label": "calcium ion binding"
}